nonsense-mediated decay complex [GO:0170010] (cellular component) References: PMID:1569946, PMID:29282598, PMID:9032286 Sources: GOC:lnp Also known as: Upf complex Definition: A highly conserved protein complex that recognises and elicits the rapid degradation of mRNAs in which an amino-acid codon has changed to a nonsense codon; occurs when the 3' end is not protected by a 3'-poly(A) tail; degradation proceeds in the 3' to 5' direction. Relationships: is a type of catalytic complex [GO:1902494]